{
  "gene": "UniProtKB:Q96AX1",
  "term_id": "UNKNOWN:0001",
  "gene_symbol": "VPS33A",
  "gene_name": "Vacuolar protein sorting-associated protein 33A",
  "term_label": "Unknown molecular function"
}